inositol monophosphate phosphatase activity [GO:0052834] (molecular function) Also known as: inositol-1(or 4)-monophosphatase activity, myo-inositol-1(or 4)-phosphate phosphohydrolase activity, L-myo-inositol-phosphate phosphatase activity, inositol phosphatase activity, inositol-phosphate phosphatase activity, myo-inositol monophosphatase activity, myo-inositol phosphatase activity, myo-inositol-phosphatase activity, myo-inositol-phosphate phosphohydrolase activity Sources: EC:3.1.3.25 Relationships: is a type of inositol phosphate phosphatase activity [GO:0052745] Definition: Catalysis of the reaction: myo-inositol phosphate + H2O = myo-inositol + phosphate. Subtypes: GO:0008934, GO:0052832, inositol monophosphate 4-phosphatase activity [GO:0052833]